{
  "gene_name": "Metalloreductase STEAP1",
  "gene": "UniProtKB:Q9UHE8",
  "term_label": "Unknown molecular function",
  "gene_symbol": "STEAP1",
  "term_id": "UNKNOWN:0001"
}